{
  "gene_name": "CCR4-NOT transcription complex subunit 11",
  "gene_symbol": "CNOT11",
  "gene": "UniProtKB:Q9UKZ1",
  "term_label": "Unknown molecular function",
  "term_id": "UNKNOWN:0001"
}